{
  "gene_symbol": "PAQR7",
  "gene": "UniProtKB:Q86WK9",
  "term_id": "GO:0048545",
  "term_label": "response to steroid hormone",
  "gene_name": "Membrane progestin receptor alpha"
}